{
  "gene_symbol": "IL13RA2",
  "gene": "UniProtKB:Q14627",
  "term_label": "cytokine receptor activity",
  "gene_name": "Interleukin-13 receptor subunit alpha-2",
  "term_id": "GO:0004896"
}